{
  "gene_name": "Bifunctional epoxide hydrolase 2",
  "term_id": "GO:0042632",
  "gene": "UniProtKB:P34913",
  "term_label": "cholesterol homeostasis",
  "gene_symbol": "EPHX2"
}